{
  "gene_name": "Tenascin-N",
  "gene_symbol": "TNN",
  "term_label": "extracellular matrix",
  "term_id": "GO:0031012",
  "gene": "UniProtKB:Q9UQP3"
}